{
  "gene": "UniProtKB:O43678",
  "gene_name": "NADH dehydrogenase [ubiquinone] 1 alpha subcomplex subunit 2",
  "gene_symbol": "NDUFA2",
  "term_label": "respiratory chain complex I",
  "term_id": "GO:0045271"
}